{
  "gene": "UniProtKB:Q9H116",
  "gene_symbol": "GZF1",
  "term_id": "GO:0000978",
  "term_label": "RNA polymerase II cis-regulatory region sequence-specific DNA binding",
  "gene_name": "GDNF-inducible zinc finger protein 1"
}